negative regulation of biosynthetic process of antibacterial peptides active against Gram-positive bacteria [GO:0002817] (biological process) Also known as: down regulation of biosynthetic process of antibacterial peptides active against Gram-positive bacteria, down-regulation of biosynthetic process of antibacterial peptides active against Gram-positive bacteria, downregulation of biosynthetic process of antibacterial peptides active against Gram-positive bacteria, inhibition of biosynthetic process of antibacterial peptides active against Gram-positive bacteria Definition: Any process that stops, prevents, or reduces the frequency, rate, or extent of biosynthesis of antibacterial peptides active against Gram-positive bacteria. Sources: GOC:add Relationships: is a type of negative regulation of antibacterial peptide biosynthetic process [GO:0002809]; is a type of GO:0002816; negatively regulates GO:0002815